{
  "term_label": "protein sequestering activity",
  "gene_symbol": "TMSB15A",
  "gene_name": "Thymosin beta-15A",
  "term_id": "GO:0140311",
  "gene": "UniProtKB:P0CG34"
}